{
  "gene_name": "Adhesion G protein-coupled receptor E1",
  "term_id": "GO:0007186",
  "gene_symbol": "ADGRE1",
  "gene": "UniProtKB:Q14246",
  "term_label": "G protein-coupled receptor signaling pathway"
}